{
  "gene_name": "Post-GPI attachment to proteins factor 6",
  "term_id": "UNKNOWN:0001",
  "gene": "UniProtKB:Q9HCN3",
  "gene_symbol": "PGAP6",
  "term_label": "Unknown molecular function"
}